positive regulation of protein localization to cilium [GO:1903566] (biological process) Definition: Any process that activates or increases the frequency, rate or extent of protein localization to cilium. Subtypes: positive regulation of protein localization to ciliary membrane [GO:1903569] Relationships: is a type of regulation of protein localization to cilium [GO:1903564]; is a type of GO:1903829; positively regulates protein localization to cilium [GO:0061512] References: PMID:22072986 Sources: GOC:TermGenie, GOC:cilia, GOC:krc, GO_REF:0000058 Also known as: up regulation of protein localization to cilium, up-regulation of protein localization to cilium, upregulation of protein localization to cilium, activation of protein localization to cilium